{
  "gene": "UniProtKB:A6NJ46",
  "term_id": "GO:0030154",
  "gene_symbol": "NKX6-3",
  "gene_name": "Homeobox protein Nkx-6.3",
  "term_label": "cell differentiation"
}